{
  "term_id": "GO:0006357",
  "gene": "UniProtKB:Q99607",
  "gene_symbol": "ELF4",
  "gene_name": "ETS-related transcription factor Elf-4",
  "term_label": "regulation of transcription by RNA polymerase II"
}